{
  "term_label": "cytoplasm",
  "term_id": "GO:0005737",
  "gene_name": "Putative heat shock 70 kDa protein 7",
  "gene_symbol": "HSPA7",
  "gene": "UniProtKB:P48741"
}